{
  "term_label": "Unknown molecular function",
  "gene": "UniProtKB:A6NFZ4",
  "gene_symbol": "FAM24A",
  "gene_name": "Protein FAM24A",
  "term_id": "UNKNOWN:0001"
}